{
  "gene": "UniProtKB:Q9HCK0",
  "gene_symbol": "ZBTB26",
  "term_label": "regulation of immune system process",
  "term_id": "GO:0002682",
  "gene_name": "Zinc finger and BTB domain-containing protein 26"
}